detection of electrical stimulus involved in magnetoreception [GO:0050970] (biological process) Definition: The series of events that contribute to magnetoception in which an electrical stimulus is received and converted into a molecular signal. The stimulus is in the form of an induced electric field resulting from movement in a magnetic field. References: PMID:15886990 Sources: GOC:ai, GOC:dos, GOC:dph, GOC:tb, Wikipedia:Magnetoception Relationships: is a type of detection of electrical stimulus involved in sensory perception [GO:0050963]; is part of GO:0050978 Also known as: magnetoception, sensory transduction of electrical stimulus, magnetoreception, detection of electrical stimulus, magnetoreception, sensory detection of electrical stimulus, magnetoreception, sensory transduction of electrical stimulus, detection of electrical stimulus during magnetoreception, sensory detection of electrical stimulus during magnetoreception, sensory transduction of electrical stimulus during magnetoreception